{
  "gene": "UniProtKB:Q9Y3C4",
  "gene_symbol": "TPRKB",
  "term_label": "tRNA threonylcarbamoyladenosine modification",
  "term_id": "GO:0002949",
  "gene_name": "EKC_KEOPS complex subunit TPRKB"
}